microtubule anchoring at spindle pole body [GO:0034631] (biological process) Subtypes: astral microtubule anchoring at mitotic spindle pole body [GO:1990734], GO:1990810 References: PMID:17486116 Sources: GOC:mah Relationships: is_a GO:0022402; is a type of microtubule anchoring at microtubule organizing center [GO:0072393]; is part of GO:0007051 Also known as: attachment of spindle microtubules to SPB, attachment of spindle microtubules to spindle pole body, microtubule anchoring at SPB Definition: Any process in which a microtubule is maintained in a specific location in a cell by attachment to a spindle pole body. Microtubules attach to spindle pole bodies at the minus end.